{
  "gene_name": "Pre-mRNA cleavage complex 2 protein Pcf11",
  "term_id": "GO:0006369",
  "gene_symbol": "PCF11",
  "term_label": "termination of RNA polymerase II transcription",
  "gene": "UniProtKB:O94913"
}